{
  "term_id": "GO:0005764",
  "gene": "UniProtKB:Q6UX65",
  "term_label": "lysosome",
  "gene_name": "DNA damage-regulated autophagy modulator protein 2",
  "gene_symbol": "DRAM2"
}